{
  "gene_symbol": "CPEB1",
  "gene": "UniProtKB:Q9BZB8",
  "term_id": "GO:0003730",
  "gene_name": "Cytoplasmic polyadenylation element-binding protein 1",
  "term_label": "mRNA 3'-UTR binding"
}